abscission [GO:0009838] (biological process) Subtypes: floral organ abscission [GO:0010227], GO:0060866, fruit abscission [GO:0060867], seed abscission [GO:0097548] Definition: The controlled shedding of a body part. Sources: ISBN:0140514031 Relationships: is a type of developmental process [GO:0032502]; is part of GO:0007275